heme oxidation [GO:0006788] (biological process) Relationships: is a type of heme metabolic process [GO:0042168]; is part of GO:0006787 Sources: GOC:mah Also known as: haem oxidation Definition: The chemical reactions and pathways resulting in the loss of electrons from one or more atoms in heme.